{
  "gene": "UniProtKB:P23759",
  "gene_name": "Paired box protein Pax-7",
  "term_id": "GO:0007399",
  "gene_symbol": "PAX7",
  "term_label": "nervous system development"
}